{
  "term_id": "GO:0007219",
  "gene": "UniProtKB:Q9NR61",
  "gene_symbol": "DLL4",
  "term_label": "Notch signaling pathway",
  "gene_name": "Delta-like protein 4"
}